{
  "gene": "UniProtKB:Q8TAM6",
  "term_id": "GO:0007015",
  "term_label": "actin filament organization",
  "gene_name": "Ermin",
  "gene_symbol": "ERMN"
}